polarity specification of anterior/posterior axis [GO:0009949] (BP) Relationships: is a type of GO:0065001; is part of anterior/posterior axis specification [GO:0009948] Sources: GOC:go_curators Definition: Any process resulting in the establishment of polarity along the anterior/posterior axis.